erythropoietin receptor activity [GO:0004900] (molecular function) Definition: Combining with erythropoietin and transmitting the signal from one side of the membrane to the other to initiate a change in cell activity. Sources: GOC:ai, GOC:signaling Relationships: is a type of cytokine receptor activity [GO:0004896]; is part of erythropoietin-mediated signaling pathway [GO:0038162]